sphere organelle [GO:0071601] (cellular component) Definition: A nuclear body that is found in the germinal vesicles of amphibian oocytes, and consist of three major parts: a remarkably spherical body about 5-10 pm in diameter, smaller spherical or nearly spherical granules on the surface, and inclusions of various sizes that strongly resemble the surface granules. The parts of the sphere organelle have distinct compositions, including splicing snRNAs and proteins. Relationships: is a type of nuclear body [GO:0016604] References: PMID:7758244, PMID:8349728